{
  "gene_name": "Small ribosomal subunit protein bS18m",
  "term_id": "GO:0003735",
  "gene": "UniProtKB:Q9Y3D5",
  "gene_symbol": "MRPS18C",
  "term_label": "structural constituent of ribosome"
}